T-helper 17 type immune response [GO:0072538] (biological process) Sources: GOC:BHF, GOC:ebc Also known as: Th17 immune response Relationships: is a type of GO:0002460 Regulation: regulated by regulation of T-helper 17 type immune response [GO:2000316]; negatively regulated by negative regulation of T-helper 17 type immune response [GO:2000317]; positively regulated by positive regulation of T-helper 17 type immune response [GO:2000318] Definition: An immune response which is associated with resistance to intracellular bacteria with a key role in inflammation and tissue injury. This immune response is associated with pathological autoimmune conditions such as multiple sclerosis, arthritis and psoriasis which is typically orchestrated by the production of particular cytokines by T-helper 17 cells, most notably interleukin-17, IL-21 and IL-22.